{
  "gene_symbol": "TPCN1",
  "gene_name": "Two pore channel protein 1",
  "term_label": "Unknown biological process",
  "term_id": "UNKNOWN:0002",
  "gene": "UniProtKB:Q9ULQ1"
}